{
  "term_id": "GO:0043162",
  "gene_name": "Vacuolar protein sorting-associated protein 37B",
  "gene_symbol": "VPS37B",
  "term_label": "ubiquitin-dependent protein catabolic process via the multivesicular body sorting pathway",
  "gene": "UniProtKB:Q9H9H4"
}